{
  "term_id": "GO:0097519",
  "gene": "UniProtKB:P15918",
  "gene_name": "V(D)J recombination-activating protein 1",
  "term_label": "DNA recombinase complex",
  "gene_symbol": "RAG1"
}